{
  "term_id": "GO:0001508",
  "gene_name": "Potassium voltage-gated channel subfamily B member 2",
  "term_label": "action potential",
  "gene": "UniProtKB:Q92953",
  "gene_symbol": "KCNB2"
}